{
  "term_id": "GO:0034440",
  "gene_name": "Polyunsaturated fatty acid lipoxygenase ALOX12",
  "term_label": "lipid oxidation",
  "gene_symbol": "ALOX12",
  "gene": "UniProtKB:P18054"
}